{
  "gene_symbol": "PLXNC1",
  "gene": "UniProtKB:O60486",
  "term_id": "GO:0002116",
  "term_label": "semaphorin receptor complex",
  "gene_name": "Plexin-C1"
}